recombinase activator activity [GO:0120230] (molecular function) Definition: Binds to and increases the activity of a recombinase. References: PMID:32414915 Sources: GOC:mah Relationships: is a type of enzyme activator activity [GO:0008047]